{
  "term_label": "mitochondrion",
  "gene_name": "Mitochondrial disaggregase",
  "gene_symbol": "CLPB",
  "term_id": "GO:0005739",
  "gene": "UniProtKB:Q9H078"
}